fructose 6-phosphate metabolic process [GO:0006002] (biological process) Sources: ISBN:0198506732 Relationships: is a type of phosphate-containing compound metabolic process [GO:0006796]; is a type of organophosphate metabolic process [GO:0019637]; is_a carbohydrate derivative metabolic process [GO:1901135] Subtypes: sucrose catabolic process to fructose-6-phosphate and glucose-6-phosphate [GO:0036008], GO:0061611 Also known as: fructose 6-phosphate metabolism Definition: The chemical reactions and pathways involving fructose 6-phosphate, also known as F6P. The D-enantiomer is an important intermediate in glycolysis, gluconeogenesis, and fructose metabolism.